toll-like receptor signaling pathway [GO:0002224] (biological process) Relationships: is a type of pattern recognition receptor signaling pathway [GO:0002221] Also known as: TLR signaling pathway, toll-like receptor signalling pathway Subtypes: GO:0002755, GO:0002756, TIRAP-dependent toll-like receptor signaling pathway [GO:0035664], toll-like receptor 21 signaling pathway [GO:0035682], toll-like receptor TLR1:TLR2 signaling pathway [GO:0038123], toll-like receptor TLR6:TLR2 signaling pathway [GO:0038124] References: PMID:12467241, PMID:12524386, PMID:12855817, PMID:15585605, PMID:15728447 Sources: GOC:add, GO_REF:0000022, ISBN:0781735149 Note: Note that the vertebrate toll-like receptors, unlike the Drosophila Toll molecule, directly bind their ligands. The Drosophila Toll molecule requires the Sptzle factor to bind microbial ligands and then the receptor in order to initiate innate immune responses. Definition: The series of molecular signals initiated by a ligand binding to a toll-like receptor of a target cell. Toll-like receptors directly bind pattern motifs from a variety of microbial sources to initiate an innate immune response. Regulation: regulated by GO:0034121; negatively regulated by GO:0034122; positively regulated by positive regulation of toll-like receptor signaling pathway [GO:0034123]